cellular response to miconazole [GO:1905308] (biological process) References: PMID:26108447 Sources: GOC:TermGenie, GO_REF:0000071 Relationships: is a type of cellular response to nitrogen compound [GO:1901699]; is a type of response to miconazole [GO:1905307] Definition: Any process that results in a change in state or activity of a cell (in terms of movement, secretion, enzyme production, gene expression, etc.) as a result of a miconazole stimulus.